ciliary rootlet [GO:0035253] (cellular component) Definition: A cytoskeleton-like structure, originating from the basal body at the proximal end of a cilium, and extending proximally toward the cell nucleus. Rootlets are typically 80-100 nm in diameter and contain cross striae distributed at regular intervals of approximately 55-70 nm. References: PMID:12427867 Sources: GOC:cilia Relationships: is_a GO:0110165; is part of GO:0005856; is part of cilium [GO:0005929] Also known as: cilial rootlet, cilium rootlet